{
  "term_label": "protein serine/threonine kinase activity",
  "gene": "UniProtKB:Q15131",
  "gene_name": "Cyclin-dependent kinase 10",
  "gene_symbol": "CDK10",
  "term_id": "GO:0004674"
}